{
  "term_id": "GO:0031902",
  "term_label": "late endosome membrane",
  "gene": "UniProtKB:Q9UJQ1",
  "gene_name": "Lysosome-associated membrane glycoprotein 5",
  "gene_symbol": "LAMP5"
}